oncogene-induced cell senescence [GO:0090402] (biological process) Relationships: is a type of GO:0090398 Sources: GOC:BHF Also known as: OIS Definition: A cellular senescence process associated with the dismantling of a cell as a response to oncogenic stress, such as the activation of the Ras oncogenic family.